{
  "term_id": "UNKNOWN:0002",
  "gene": "UniProtKB:O15084",
  "gene_name": "Serine_threonine-protein phosphatase 6 regulatory ankyrin repeat subunit A",
  "term_label": "Unknown biological process",
  "gene_symbol": "ANKRD28"
}